naringenin 7-O-methyltransferase activity [GO:0102766] (molecular function) Relationships: is_a methyltransferase activity [GO:0008168] Sources: EC:2.1.1.232, GOC:pz Definition: Catalysis of the reaction: (S)-naringenin(1-) + S-adenosyl-L-methionine = sakuranetin + S-adenosyl-L-homocysteine + H+.